{
  "gene": "UniProtKB:P15382",
  "term_id": "GO:0086091",
  "gene_symbol": "KCNE1",
  "term_label": "regulation of heart rate by cardiac conduction",
  "gene_name": "Potassium voltage-gated channel subfamily E member 1"
}